{
  "gene_name": "Guanine nucleotide-binding protein subunit alpha-14",
  "term_id": "GO:0001664",
  "gene_symbol": "GNA14",
  "term_label": "G protein-coupled receptor binding",
  "gene": "UniProtKB:O95837"
}